{
  "term_id": "GO:0000981",
  "gene": "UniProtKB:Q9GZZ0",
  "gene_symbol": "HOXD1",
  "term_label": "DNA-binding transcription factor activity, RNA polymerase II-specific",
  "gene_name": "Homeobox protein Hox-D1"
}